{
  "gene_symbol": "KRTAP4-16",
  "gene_name": "Putative keratin-associated protein 4-16",
  "term_label": "Unknown molecular function",
  "term_id": "UNKNOWN:0001",
  "gene": "UniProtKB:G5E9R7"
}